{
  "gene_name": "Beta-crystallin A4",
  "gene": "UniProtKB:P53673",
  "gene_symbol": "CRYBA4",
  "term_id": "UNKNOWN:0003",
  "term_label": "Unknown cellular component"
}